{
  "gene_name": "Sorbin and SH3 domain-containing protein 2",
  "term_id": "GO:0045202",
  "term_label": "synapse",
  "gene_symbol": "SORBS2",
  "gene": "UniProtKB:O94875"
}